{
  "gene": "UniProtKB:Q6ZRT6",
  "term_label": "Unknown cellular component",
  "gene_symbol": "PRR23B",
  "gene_name": "Proline-rich protein 23B",
  "term_id": "UNKNOWN:0003"
}